pyrimidine ribonucleoside diphosphate metabolic process [GO:0009193] (biological process) Subtypes: pyrimidine ribonucleoside diphosphate biosynthetic process [GO:0009194], pyrimidine ribonucleoside diphosphate catabolic process [GO:0009195], GO:0046043, UDP metabolic process [GO:0046048], CDP metabolic process [GO:0046704] Sources: GOC:go_curators, ISBN:0198506732 Definition: The chemical reactions and pathways involving pyrimidine ribonucleoside diphosphate, a compound consisting of a pyrimidine base linked to a ribose sugar esterified with diphosphate on the sugar. Relationships: is a type of pyrimidine nucleoside diphosphate metabolic process [GO:0009138]; is a type of ribonucleoside diphosphate metabolic process [GO:0009185] Also known as: pyrimidine ribonucleoside diphosphate metabolism